3-chloroallyl aldehyde dehydrogenase activity [GO:0004028] (molecular function) Relationships: is a type of oxidoreductase activity, acting on the aldehyde or oxo group of donors, NAD or NADP as acceptor [GO:0016620] Definition: Catalysis of the reaction: 3-chloroallyl aldehyde + H2O = 2 H+ + 2 e- + 3-chloroacrylic acid. Sources: GOC:curators